{
  "gene_name": "Zinc transporter ZIP10",
  "gene_symbol": "SLC39A10",
  "gene": "UniProtKB:Q9ULF5",
  "term_label": "plasma membrane",
  "term_id": "GO:0005886"
}